{
  "gene_name": "Transcription factor SOX-9",
  "gene_symbol": "SOX9",
  "gene": "UniProtKB:P48436",
  "term_label": "oligodendrocyte differentiation",
  "term_id": "GO:0048709"
}